{
  "gene": "UniProtKB:A6NM62",
  "gene_symbol": "LRRC53",
  "term_label": "plasma membrane",
  "term_id": "GO:0005886",
  "gene_name": "Leucine-rich repeat-containing protein 53"
}